{
  "gene_name": "Semaphorin-5B",
  "term_label": "semaphorin receptor binding",
  "gene": "UniProtKB:Q9P283",
  "term_id": "GO:0030215",
  "gene_symbol": "SEMA5B"
}